interleukin-15 receptor activity [GO:0042010] (molecular function) Relationships: is a type of cytokine receptor activity [GO:0004896]; is part of GO:0035723; has part GO:0042009 Also known as: IL-15 receptor activity, IL-15R Sources: GOC:jl, GOC:signaling Definition: Combining with interleukin-15 and transmitting the signal from one side of the membrane to the other to initiate a change in cell activity.